{
  "gene_name": "N-acetylglutamate synthase, mitochondrial",
  "term_label": "L-glutamate N-acetyltransferase activity",
  "term_id": "GO:0004042",
  "gene": "UniProtKB:Q8N159",
  "gene_symbol": "NAGS"
}